{
  "term_label": "Unknown molecular function",
  "term_id": "UNKNOWN:0001",
  "gene_symbol": "ILDR2",
  "gene": "UniProtKB:Q71H61",
  "gene_name": "Immunoglobulin-like domain-containing receptor 2"
}